{
  "gene": "UniProtKB:P30273",
  "gene_symbol": "FCER1G",
  "term_label": "Fc-gamma receptor signaling pathway",
  "gene_name": "High affinity immunoglobulin epsilon receptor subunit gamma",
  "term_id": "GO:0038094"
}